{
  "term_id": "GO:0005886",
  "gene_name": "Membrane-spanning 4-domains subfamily A member 12",
  "gene_symbol": "MS4A12",
  "term_label": "plasma membrane",
  "gene": "UniProtKB:Q9NXJ0"
}